cephalosporin biosynthetic process [GO:0043646] (BP) Definition: The chemical reactions and pathways resulting in the formation of a cephalosporin, any of large class of tetracyclic triterpene broad-spectrum antibiotics similar both chemically and in their mode of action to penicillin, first isolated from the culture filtrates of mediterranean fungus acremonium (cephalosporium acremonium), and effective against gram-positive bacteria. Sources: GOC:jl, Wikipedia:Cephalosporin Relationships: is a type of beta-lactam antibiotic biosynthetic process [GO:0030654]; is a type of sulfur compound biosynthetic process [GO:0044272] Subtypes: GO:1901268